acetylation-dependent protein binding [GO:0140033] (molecular function) References: PMID:26060076 Note: This term should only be used when the binding is shown to require acetylation of the target protein: the interaction needs to be tested with and without the PTM. The binding does not need to be at the site of acetylation. It may be that the acetylation causes a conformational change that allows binding of the protein to another region; this type of acetylation-dependent protein binding is valid for annotation to this term. Relationships: is a type of modification-dependent protein binding [GO:0140030] Definition: Binding to a protein upon acetylation of the target protein.